glucose 1-dehydrogenase (NADP+) activity [GO:0047935] (molecular function) Sources: EC:1.1.1.119, MetaCyc:GLUCOSE-1-DEHYDROGENASE-NADP+-RXN Relationships: is a type of GO:0047936 Also known as: D-glucose:NADP+ 1-oxidoreductase activity, NADP-dependent glucose dehydrogenase activity, NADP-linked aldohexose dehydrogenase activity, nicotinamide adenine dinucleotide phosphate-linked aldohexose dehydrogenase activity Definition: Catalysis of the reaction: D-glucose + NADP+ = D-glucono-1,5-lactone + NADPH.